{
  "term_label": "Unknown cellular component",
  "gene_name": "Transmembrane protein 200A",
  "term_id": "UNKNOWN:0003",
  "gene": "UniProtKB:Q86VY9",
  "gene_symbol": "TMEM200A"
}